smooth muscle cell apoptotic process [GO:0034390] (biological process) Definition: Any apoptotic process in a smooth muscle cell. Smooth muscle consists of non-striated, elongated, spindle-shaped cell found lining the digestive tract, uterus, and blood vessels. Relationships: is a type of muscle cell apoptotic process [GO:0010657] Regulation: regulated by regulation of smooth muscle cell apoptotic process [GO:0034391]; negatively regulated by GO:0034392; positively regulated by positive regulation of smooth muscle cell apoptotic process [GO:0034393] Subtypes: vascular associated smooth muscle cell apoptotic process [GO:1905288] Sources: CL:0000192, GOC:BHF, GOC:mah, GOC:mtg_apoptosis, GOC:rl Also known as: SMC apoptosis, apoptosis of smooth muscle cells, programmed cell death of smooth muscle cells by apoptosis, programmed cell death, smooth muscle cells, smooth muscle cell programmed cell death by apoptosis, smooth muscle cell apoptosis